{
  "gene": "UniProtKB:P51956",
  "gene_name": "Serine_threonine-protein kinase Nek3",
  "term_id": "UNKNOWN:0003",
  "gene_symbol": "NEK3",
  "term_label": "Unknown cellular component"
}